GUC codon-amino acid adaptor activity [GO:0033450] (molecular function) Definition: A triplet codon-amino acid adaptor activity that recognizes a GUC codon. Sources: GOC:mah Also known as: GTC codon-amino acid adaptor activity, valine tRNA Note: Note that in the standard genetic code, GTC codes for valine. Relationships: is a type of GO:0030533